{
  "gene": "UniProtKB:P05093",
  "gene_name": "Steroid 17-alpha-hydroxylase_17,20 lyase",
  "gene_symbol": "CYP17A1",
  "term_label": "Unknown cellular component",
  "term_id": "UNKNOWN:0003"
}